{
  "term_id": "GO:0005789",
  "term_label": "endoplasmic reticulum membrane",
  "gene_symbol": "ALG12",
  "gene_name": "Dol-P-Man:Man(7)GlcNAc(2)-PP-Dol alpha-1,6-mannosyltransferase",
  "gene": "UniProtKB:Q9BV10"
}